{
  "gene_symbol": "DNASE1L3",
  "gene_name": "Deoxyribonuclease gamma",
  "term_id": "GO:0003677",
  "gene": "UniProtKB:Q13609",
  "term_label": "DNA binding"
}